{
  "gene_symbol": "GPR18",
  "gene_name": "N-arachidonyl glycine receptor",
  "term_label": "plasma membrane",
  "term_id": "GO:0005886",
  "gene": "UniProtKB:Q14330"
}